{
  "gene_symbol": "SLC25A15",
  "term_id": "GO:0005739",
  "term_label": "mitochondrion",
  "gene": "UniProtKB:Q9Y619",
  "gene_name": "Mitochondrial ornithine transporter 1"
}